pancreatic A cell fate commitment [GO:0003326] (biological process) Relationships: is a type of epithelial cell fate commitment [GO:0072148]; is part of pancreatic A cell differentiation [GO:0003310] Sources: GOC:dph Definition: The commitment of a cell to a pancreatic A cell and its capacity to differentiate into a pancreatic A cell. A pancreatic A cell is a cell in the pancreas that secretes glucagon.